{
  "gene_symbol": "ENHO",
  "term_label": "positive regulation of Notch signaling pathway",
  "gene_name": "Adropin",
  "term_id": "GO:0045747",
  "gene": "UniProtKB:Q6UWT2"
}